{
  "gene_name": "Prostaglandin E synthase 2",
  "gene_symbol": "PTGES2",
  "term_label": "prostaglandin-E synthase activity",
  "term_id": "GO:0050220",
  "gene": "UniProtKB:Q9H7Z7"
}